{
  "gene_symbol": "HPCAL1",
  "gene": "UniProtKB:P37235",
  "gene_name": "Hippocalcin-like protein 1",
  "term_id": "GO:0009966",
  "term_label": "regulation of signal transduction"
}